{
  "term_id": "GO:0004867",
  "term_label": "serine-type endopeptidase inhibitor activity",
  "gene": "UniProtKB:P01009",
  "gene_symbol": "SERPINA1",
  "gene_name": "Alpha-1-antitrypsin"
}